{
  "gene_name": "BTB_POZ domain-containing protein KCTD2",
  "term_label": "cullin family protein binding",
  "gene_symbol": "KCTD2",
  "term_id": "GO:0097602",
  "gene": "UniProtKB:Q14681"
}